{
  "gene_name": "Ribitol-5-phosphate transferase FKTN",
  "term_label": "Unknown molecular function",
  "term_id": "UNKNOWN:0001",
  "gene_symbol": "FKTN",
  "gene": "UniProtKB:O75072"
}